glycine dehydrogenase (cytochrome) activity [GO:0047959] (molecular function) Also known as: glycine-cytochrome c reductase activity, glycine:ferricytochrome-c oxidoreductase (deaminating), reductase, glycine-cytochrome c Definition: Catalysis of the reaction: glycine + H2O + 2 ferricytochrome c = glyoxylate + NH3 + 2 ferrocytochrome c. Relationships: is a type of oxidoreductase activity, acting on the CH-NH2 group of donors, cytochrome as acceptor [GO:0016640] Sources: EC:1.4.2.1, MetaCyc:GLYCINE-DEHYDROGENASE-CYTOCHROME-RXN